{
  "gene": "UniProtKB:Q14BN4",
  "gene_name": "Sarcolemmal membrane-associated protein",
  "term_id": "UNKNOWN:0001",
  "term_label": "Unknown molecular function",
  "gene_symbol": "SLMAP"
}